{
  "term_label": "establishment or maintenance of epithelial cell apical/basal polarity",
  "gene": "UniProtKB:Q5IJ48",
  "gene_name": "Protein crumbs homolog 2",
  "term_id": "GO:0045197",
  "gene_symbol": "CRB2"
}